{
  "gene_symbol": "EMSY",
  "gene_name": "BRCA2-interacting transcriptional repressor EMSY",
  "term_label": "Unknown biological process",
  "gene": "UniProtKB:Q7Z589",
  "term_id": "UNKNOWN:0002"
}